{
  "gene_symbol": "SHBG",
  "term_id": "GO:0005497",
  "term_label": "androgen binding",
  "gene": "UniProtKB:P04278",
  "gene_name": "Sex hormone-binding globulin"
}